{
  "gene": "UniProtKB:Q9HAW8",
  "gene_name": "UDP-glucuronosyltransferase 1A10",
  "term_label": "cellular response to glucocorticoid stimulus",
  "gene_symbol": "UGT1A10",
  "term_id": "GO:0071385"
}